{
  "term_id": "UNKNOWN:0002",
  "term_label": "Unknown biological process",
  "gene_name": "Inactive serine protease PAMR1",
  "gene_symbol": "PAMR1",
  "gene": "UniProtKB:Q6UXH9"
}